pyridine nucleotide biosynthetic process [GO:0019363] (biological process) Also known as: pyridine nucleotide anabolism, pyridine nucleotide biosynthesis, pyridine nucleotide formation, pyridine nucleotide synthesis Relationships: is a type of nucleotide biosynthetic process [GO:0009165]; is a type of pyridine-containing compound biosynthetic process [GO:0072525] Definition: The chemical reactions and pathways resulting in the formation of a pyridine nucleotide, a nucleotide characterized by a pyridine derivative as a nitrogen base. Sources: GOC:jl, GOC:pde, GOC:vw Subtypes: nicotinate nucleotide biosynthetic process [GO:0019357], nicotinamide nucleotide biosynthetic process [GO:0019359], GO:0019365